{
  "gene_symbol": "NTAN1",
  "term_id": "GO:0006511",
  "gene_name": "Protein N-terminal asparagine amidohydrolase",
  "term_label": "ubiquitin-dependent protein catabolic process",
  "gene": "UniProtKB:Q96AB6"
}